{
  "gene_name": "Carboxypeptidase A6",
  "term_id": "GO:0004181",
  "gene": "UniProtKB:Q8N4T0",
  "gene_symbol": "CPA6",
  "term_label": "metallocarboxypeptidase activity"
}